{
  "gene": "UniProtKB:P0DPD6",
  "gene_name": "Endothelin-converting enzyme 2",
  "term_id": "GO:0004222",
  "gene_symbol": "ECE2",
  "term_label": "metalloendopeptidase activity"
}